{
  "gene_symbol": "BICDL2",
  "term_label": "Golgi to secretory granule transport",
  "gene": "UniProtKB:A1A5D9",
  "gene_name": "BICD family-like cargo adapter 2",
  "term_id": "GO:0055107"
}